{
  "term_id": "GO:0004725",
  "gene_symbol": "DUSP23",
  "gene_name": "Dual specificity protein phosphatase 23",
  "gene": "UniProtKB:Q9BVJ7",
  "term_label": "protein tyrosine phosphatase activity"
}